lipid hydroperoxide transport [GO:1901373] (BP) Relationships: is a type of lipid transport [GO:0006869] Definition: The directed movement of a lipid hydroperoxide into, out of or within a cell, or between cells, by means of some agent such as a transporter or pore. Sources: GOC:TermGenie